{
  "term_id": "GO:0004674",
  "gene": "UniProtKB:Q9BXA6",
  "term_label": "protein serine/threonine kinase activity",
  "gene_name": "Testis-specific serine_threonine-protein kinase 6",
  "gene_symbol": "TSSK6"
}